{
  "gene_name": "Serum amyloid A-2 protein",
  "term_id": "UNKNOWN:0003",
  "gene_symbol": "SAA2",
  "gene": "UniProtKB:P0DJI9",
  "term_label": "Unknown cellular component"
}